{
  "term_id": "GO:0005789",
  "term_label": "endoplasmic reticulum membrane",
  "gene": "UniProtKB:P78383",
  "gene_name": "Solute carrier family 35 member B1",
  "gene_symbol": "SLC35B1"
}